{
  "term_id": "GO:0033962",
  "gene": "UniProtKB:C9JE40",
  "gene_symbol": "PATL2",
  "gene_name": "Protein PAT1 homolog 2",
  "term_label": "P-body assembly"
}